{
  "gene_name": "Excitatory amino acid transporter 5",
  "term_label": "glutamate:sodium symporter activity",
  "term_id": "GO:0015501",
  "gene_symbol": "SLC1A7",
  "gene": "UniProtKB:O00341"
}